dCMP salvage [GO:0006239] (biological process) Sources: GOC:jl Definition: Any process that generates dCMP, deoxycytidine monophosphate from derivatives of it, without de novo synthesis. Also known as: deoxycytidine monophosphate salvage Relationships: is a type of pyrimidine deoxyribonucleotide salvage [GO:0010139]; is_a dCMP biosynthetic process [GO:0046064]